{
  "gene_name": "Nitric oxide synthase 1",
  "term_id": "GO:0050660",
  "gene_symbol": "NOS1",
  "term_label": "flavin adenine dinucleotide binding",
  "gene": "UniProtKB:P29475"
}